{
  "gene": "UniProtKB:Q92985",
  "gene_symbol": "IRF7",
  "term_label": "immune system process",
  "gene_name": "Interferon regulatory factor 7",
  "term_id": "GO:0002376"
}